{
  "gene": "UniProtKB:Q92499",
  "gene_name": "ATP-dependent RNA helicase DDX1",
  "term_label": "Unknown cellular component",
  "gene_symbol": "DDX1",
  "term_id": "UNKNOWN:0003"
}